myo-inositol transport [GO:0015798] (biological process) Subtypes: myo-inositol import across plasma membrane [GO:1904679] Sources: GOC:ai Relationships: is a type of GO:0015850 Also known as: vitamin Bh transport Definition: The directed movement of myo-inositol into, out of or within a cell, or between cells, by means of some agent such as a transporter or pore. Myo-inositol is 1,2,3,4,5/4,6-cyclohexanehexol, a growth factor for animals and microorganisms.